{
  "term_label": "Rac protein signal transduction",
  "gene_symbol": "GARRE1",
  "gene": "UniProtKB:O15063",
  "gene_name": "Granule associated Rac and RHOG effector protein 1",
  "term_id": "GO:0016601"
}